{
  "gene_name": "Cytochrome P450 11B1, mitochondrial",
  "gene_symbol": "CYP11B1",
  "gene": "UniProtKB:P15538",
  "term_id": "GO:0071375",
  "term_label": "cellular response to peptide hormone stimulus"
}